{
  "gene_symbol": "LBHD1",
  "term_id": "UNKNOWN:0001",
  "gene_name": "LBH domain-containing protein 1",
  "gene": "UniProtKB:Q9BQE6",
  "term_label": "Unknown molecular function"
}